{
  "term_id": "GO:0030020",
  "term_label": "extracellular matrix structural constituent conferring tensile strength",
  "gene": "UniProtKB:P02462",
  "gene_symbol": "COL4A1",
  "gene_name": "Collagen alpha-1(IV) chain"
}